{
  "gene_symbol": "SLC52A1",
  "term_label": "riboflavin transmembrane transporter activity",
  "gene_name": "Solute carrier family 52, riboflavin transporter, member 1",
  "term_id": "GO:0032217",
  "gene": "UniProtKB:Q9NWF4"
}